clathrin-coated endocytic vesicle [GO:0045334] (cellular component) Definition: A clathrin-coated, membrane-bounded intracellular vesicle formed by invagination of the plasma membrane around an extracellular substance. Sources: GOC:go_curators Relationships: is a type of GO:0030136; is a type of endocytic vesicle [GO:0030139] Subtypes: clathrin-coated phagocytic vesicle [GO:0045336]